{
  "term_id": "GO:0005730",
  "term_label": "nucleolus",
  "gene": "UniProtKB:P46087",
  "gene_symbol": "NOP2",
  "gene_name": "Probable 28S rRNA (cytosine(4447)-C(5))-methyltransferase"
}